tricellular tight junction [GO:0061689] (cellular component) References: PMID:22520461, PMID:25822906 Sources: GOC:dk, GOC:dph Definition: An specialized occluding junction where three epithelial cells meet. It is composed of a branching network of sealing strands that run perpendicularly to the bicellular tight junction at the point of contact between three epithelial cells in an epithelial sheet. Relationships: is a type of tight junction [GO:0070160]